neuron fate commitment [GO:0048663] (biological process) Relationships: is a type of cell fate commitment [GO:0045165]; is part of neuron differentiation [GO:0030182] Also known as: neuron lineage restriction, neuronal lineage restriction Definition: The process in which the developmental fate of a cell becomes restricted such that it will develop into a neuron. Sources: GOC:dph Subtypes: pancreatic D cell fate commitment [GO:0003328], noradrenergic neuron fate commitment [GO:0003359], forebrain neuron fate commitment [GO:0021877], GO:0021890, cerebral cortex GABAergic interneuron fate commitment [GO:0021893], somatic motor neuron fate commitment [GO:0021917], photoreceptor cell fate commitment [GO:0046552], GO:0060120, GO:0060163, ventral spinal cord interneuron fate commitment [GO:0060579], cardiac neuron fate commitment [GO:0060960]